{
  "gene": "UniProtKB:P17735",
  "gene_name": "Tyrosine aminotransferase",
  "term_label": "L-phenylalanine catabolic process",
  "gene_symbol": "TAT",
  "term_id": "GO:0006559"
}